{
  "gene_name": "Gap junction beta-2 protein",
  "gene_symbol": "GJB2",
  "term_id": "GO:0005922",
  "gene": "UniProtKB:P29033",
  "term_label": "connexin complex"
}